symbiont-mediated suppression of host reactive oxygen species generation [GO:0141083] (biological process) Relationships: is a type of GO:0044068; is a type of symbiont-mediated perturbation of host defense response [GO:0052031] References: PMID:27473656, PMID:31375544 Definition: A process in which a symbiont interferes with, inhibits or disrupts the host signal transduction pathways leading to the production of reactive oxygen species as part of the host innate immune response. The host is defined as the larger of the organisms involved in a symbiotic interaction. Also known as: inhibition by organism of defense-related host active oxygen species production